{
  "gene": "UniProtKB:Q9BSJ1",
  "term_label": "ubiquitin protein ligase activity",
  "gene_symbol": "TRIM51",
  "term_id": "GO:0061630",
  "gene_name": "Tripartite motif-containing protein 51"
}